{
  "term_label": "immune response-inhibiting cell surface receptor signaling pathway",
  "gene": "UniProtKB:Q6PI73",
  "term_id": "GO:0002767",
  "gene_symbol": "LILRA6",
  "gene_name": "Leukocyte immunoglobulin-like receptor subfamily A member 6"
}